{
  "gene_symbol": "APOBEC3F",
  "term_label": "RNA binding",
  "term_id": "GO:0003723",
  "gene": "UniProtKB:Q8IUX4",
  "gene_name": "DNA dC-dU-editing enzyme APOBEC-3F"
}